{
  "gene": "UniProtKB:Q5JT25",
  "gene_symbol": "RAB41",
  "term_label": "endomembrane system",
  "term_id": "GO:0012505",
  "gene_name": "Ras-related protein Rab-41"
}